{
  "gene_name": "Myelin protein zero-like protein 2",
  "gene": "UniProtKB:O60487",
  "term_label": "plasma membrane",
  "term_id": "GO:0005886",
  "gene_symbol": "MPZL2"
}